Wnt signaling pathway involved in heart development [GO:0003306] (biological process) Relationships: is a type of GO:0016055; is a type of cell surface receptor signaling pathway involved in heart development [GO:0061311] Subtypes: canonical Wnt signaling pathway involved in heart development [GO:0061316], non-canonical Wnt signaling pathway involved in heart development [GO:0061341] Sources: GOC:mtg_heart Also known as: Wnt receptor signaling pathway involved in heart development, Wnt receptor signalling pathway involved in heart development, Wnt-activated signaling pathway involved in heart development Definition: The series of molecular signals initiated by binding of Wnt protein to a receptor on the surface of the target cell, resulting a change in cell state that contributes to the progression of the heart over time. Regulation: regulated by GO:0003307; negatively regulated by negative regulation of Wnt signaling pathway involved in heart development [GO:0003308]